response to butyrate [GO:1903544] (biological process) Relationships: is a type of GO:0070542 Definition: Any process that results in a change in state or activity of a cell or an organism (in terms of movement, secretion, enzyme production, gene expression, etc.) as a result of a butyrate stimulus. Subtypes: cellular response to butyrate [GO:1903545] References: PMID:9734870 Sources: GOC:TermGenie, GOC:mr, GO_REF:0000071